{
  "gene_name": "ELL-associated factor 1",
  "term_label": "transcription elongation factor complex",
  "term_id": "GO:0008023",
  "gene_symbol": "EAF1",
  "gene": "UniProtKB:Q96JC9"
}